deoxyguanosine kinase activity [GO:0004138] (molecular function) Also known as: (dihydroxypropoxymethyl)guanine kinase activity, 2'-deoxyguanosine kinase activity, ATP:deoxyguanosine 5'-phosphotransferase activity, NTP-deoxyguanosine 5'-phosphotransferase activity, deoxyguanosine kinase (phosphorylating) Sources: EC:2.7.1.113, RHEA:19201 Relationships: is a type of deoxynucleoside kinase activity [GO:0019136] Definition: Catalysis of the reaction: 2'-deoxyguanosine + ATP = ADP + dGMP + 2 H+.